{
  "term_label": "neuron projection",
  "gene_name": "Teneurin-4",
  "gene": "UniProtKB:Q6N022",
  "term_id": "GO:0043005",
  "gene_symbol": "TENM4"
}